{
  "term_label": "cilium movement",
  "term_id": "GO:0003341",
  "gene_name": "Dynein axonemal intermediate chain 1",
  "gene_symbol": "DNAI1",
  "gene": "UniProtKB:Q9UI46"
}